{
  "gene": "UniProtKB:P43115",
  "term_id": "GO:0005886",
  "gene_name": "Prostaglandin E2 receptor EP3 subtype",
  "gene_symbol": "PTGER3",
  "term_label": "plasma membrane"
}